snoRNA splicing [GO:0034247] (biological process) Definition: The process of removing sections of a primary snoRNA transcript to remove sequences not present in the mature form of the snoRNA and joining the remaining sections to form the mature form of the snoRNA. Sources: GOC:mah Relationships: is a type of RNA splicing [GO:0008380]; is a type of sno(s)RNA processing [GO:0043144]